regulation of aortic smooth muscle cell differentiation [GO:1904829] (BP) Subtypes: GO:1904830, positive regulation of aortic smooth muscle cell differentiation [GO:1904831] Definition: Any process that modulates the frequency, rate or extent of aortic smooth muscle cell differentiation. References: PMID:22034194 Sources: GOC:BHF, GOC:BHF_miRNA, GOC:TermGenie, GOC:rph, GO_REF:0000058 Relationships: is a type of regulation of vascular associated smooth muscle cell differentiation [GO:1905063]; regulates aortic smooth muscle cell differentiation [GO:0035887]